{
  "gene": "UniProtKB:P55055",
  "term_id": "GO:0050728",
  "gene_name": "Oxysterols receptor LXR-beta",
  "gene_symbol": "NR1H2",
  "term_label": "negative regulation of inflammatory response"
}